benzene-containing compound metabolic process [GO:0042537] (biological process) Relationships: is a type of GO:0008152 Sources: GOC:jl Subtypes: salicylic acid metabolic process [GO:0009696], cinnamic acid metabolic process [GO:0009803], stilbene biosynthetic process [GO:0009811], phenylacetate catabolic process [GO:0010124], benzoate metabolic process [GO:0018874], benzonitrile metabolic process [GO:0018876], GO:0018879, GO:0018880, GO:0018881, 4-carboxy-4'-sulfoazobenzene metabolic process [GO:0018887], 2,4-dichlorophenoxyacetic acid metabolic process [GO:0018901], benzene metabolic process [GO:0018910], 1,2,4-trichlorobenzene catabolic process [GO:0018911], chlorobenzene catabolic process [GO:0018914], ethylbenzene catabolic process [GO:0018915], nitrobenzene metabolic process [GO:0018916], GO:0018922, mandelate metabolic process [GO:0018924], phthalate metabolic process [GO:0018963], styrene metabolic process [GO:0018966], toluene metabolic process [GO:0018970], 1,1,1-trichloro-2,2-bis-(4-chlorophenyl)ethane metabolic process [GO:0018977], vanillin metabolic process [GO:0018982], 1,4-dichlorobenzene catabolic process [GO:0019261], pentachlorophenol catabolic process [GO:0019338], 3-phenylpropionate catabolic process [GO:0019380], GO:0019396, phenylmercury acetate catabolic process [GO:0019506], 4-toluenecarboxylate catabolic process [GO:0019612], GO:0031147, sinapate biosynthetic process [GO:0033497], GO:0042184, GO:0042854, anthranilate metabolic process [GO:0043420], orcinol biosynthetic process [GO:0046197], 2,4,5-trichlorophenoxyacetic acid catabolic process [GO:0046228], 2-aminobenzenesulfonate catabolic process [GO:0046230], GO:0046272, methylgallate catabolic process [GO:0046276], methylgallate biosynthetic process [GO:0046277], 3,4-dihydroxybenzoate metabolic process [GO:0046278], GO:0046298, 2-chloro-N-isopropylacetanilide catabolic process [GO:0046302], para-aminobenzoic acid metabolic process [GO:0046482], GO:0070189, toluene-containing compound catabolic process [GO:0072491], gerfelin catabolic process [GO:1900577], gerfelin biosynthetic process [GO:1900578], GO:1900583, GO:1900584, GO:1900813, GO:1901168, 3-chlorocatechol biosynthetic process [GO:1901169], (-)-pinoresinol metabolic process [GO:1901598], olivetolic acid biosynthetic process [GO:1901697], GO:1901782, p-cumate biosynthetic process [GO:1901783], p-cresol biosynthetic process [GO:1901786], homogentisate catabolic process [GO:1902000], (+)-pinoresinol catabolic process [GO:1902125], (+)-pinoresinol biosynthetic process [GO:1902126] Also known as: benzene and derivative metabolic process, benzene and derivative metabolism, benzene-containing compound metabolism Definition: The chemical reactions and pathways involving benzene, C6H6, a volatile, very inflammable liquid, contained in the naphtha produced by the destructive distillation of coal, from which it is separated by fractional distillation, or any of its derivatives.